{
  "gene": "UniProtKB:P55060",
  "term_id": "GO:0005049",
  "gene_symbol": "CSE1L",
  "term_label": "nuclear export signal receptor activity",
  "gene_name": "Exportin-2"
}